{
  "gene_symbol": "OR5D3",
  "term_id": "UNKNOWN:0003",
  "gene": "UniProtKB:A0A2R8Y4L6",
  "term_label": "Unknown cellular component",
  "gene_name": "Olfactory receptor"
}